{
  "gene_name": "Putative protein CASTOR3P",
  "term_label": "Unknown molecular function",
  "term_id": "UNKNOWN:0001",
  "gene_symbol": "CASTOR3P",
  "gene": "UniProtKB:Q8NAP1"
}